{
  "gene_name": "Pleckstrin homology domain-containing family N member 1",
  "term_label": "mitochondrial membrane",
  "term_id": "GO:0031966",
  "gene": "UniProtKB:Q494U1",
  "gene_symbol": "PLEKHN1"
}